{
  "term_id": "GO:0046703",
  "gene": "UniProtKB:Q6H3X3",
  "term_label": "natural killer cell lectin-like receptor binding",
  "gene_symbol": "RAET1G",
  "gene_name": "UL-16 binding protein 5"
}